{
  "gene_symbol": "OR1J4",
  "term_label": "plasma membrane",
  "term_id": "GO:0005886",
  "gene": "UniProtKB:Q8NGS1",
  "gene_name": "Olfactory receptor 1J4"
}